anterior/posterior axis specification [GO:0009948] (biological process) Relationships: is a type of axis specification [GO:0009798]; is part of anterior/posterior pattern specification [GO:0009952] Also known as: anterior/posterior axis determination Sources: GOC:dph, GOC:go_curators, GOC:tb Subtypes: oocyte anterior/posterior axis specification [GO:0007314], anterior/posterior axis specification, embryo [GO:0008595], GO:0032525 Definition: The establishment, maintenance and elaboration of the anterior/posterior axis. The anterior-posterior axis is defined by a line that runs from the head or mouth of an organism to the tail or opposite end of the organism.